{
  "term_id": "GO:0034982",
  "gene_name": "AFG3-like protein 2",
  "term_label": "mitochondrial protein processing",
  "gene": "UniProtKB:Q9Y4W6",
  "gene_symbol": "AFG3L2"
}